{
  "term_label": "proteasome-mediated ubiquitin-dependent protein catabolic process",
  "gene_name": "E3 ubiquitin-protein transferase MAEA",
  "term_id": "GO:0043161",
  "gene": "UniProtKB:Q7L5Y9",
  "gene_symbol": "MAEA"
}